glucosylglycerol biosynthetic process [GO:0051473] (biological process) Relationships: is a type of glycoside biosynthetic process [GO:0016138]; is a type of alditol biosynthetic process [GO:0019401]; is a type of GO:0051472 Also known as: glucosylglycerol anabolism, glucosylglycerol biosynthesis, glucosylglycerol formation, glucosylglycerol synthesis Sources: GOC:ai Definition: The chemical reactions and pathways resulting in the formation of glucosylglycerol, alpha-D-glucopyranosyl-alpha-(1,2)-glycerol.